{
  "gene_name": "Uncharacterized protein",
  "gene_symbol": "A0A0G2JLW4",
  "term_label": "Unknown biological process",
  "term_id": "UNKNOWN:0002",
  "gene": "UniProtKB:A0A0G2JLW4"
}